patulin biosynthetic process [GO:0140723] (biological process) Definition: The chemical reactions and pathways resulting in the formation of patulin, an acetate-derived tetraketide mycotoxin produced by several fungal species that shows antimicrobial properties against several bacteria. References: PMID:25120234, PMID:30680886 Also known as: patulin anabolism, patulin biosynthesis, patulin formation, patulin synthesis Relationships: is a type of polyketide biosynthetic process [GO:0030639]; is a type of mycotoxin biosynthetic process [GO:0043386]; is a type of alcohol biosynthetic process [GO:0046165]; is a type of GO:1901336 Regulation: positively regulated by GO:0140724